{
  "gene": "UniProtKB:Q8IYX7",
  "term_id": "GO:0008017",
  "gene_name": "Stabilizer of axonemal microtubules 1",
  "term_label": "microtubule binding",
  "gene_symbol": "SAXO1"
}